{
  "gene": "UniProtKB:Q9Y3F4",
  "term_label": "spliceosomal snRNP assembly",
  "gene_name": "Serine-threonine kinase receptor-associated protein",
  "gene_symbol": "STRAP",
  "term_id": "GO:0000387"
}